apical constriction involved in ventral furrow formation [GO:0110072] (biological process) Definition: The actin-mediated process that results in contraction of the apical end of a polarized columnar epithelial cell, contributing to formation of a ventral indentation (furrow) from the blastoderm epithelium, which is internalized to form a tube in the interior of the embryo, marking the start of gastrulation. References: PMID:28495958 Sources: GOC:ha Relationships: is a type of apical constriction involved in gastrulation [GO:0003384]; is part of ventral furrow formation [GO:0007370] Regulation: regulated by regulation of apical constriction involved in ventral furrow formation [GO:0110073]; positively regulated by positive regulation of apical constriction involved in ventral furrow formation [GO:0110074]